positive regulation of pyruvate decarboxylation to acetyl-CoA [GO:0140176] (biological process) References: PMID:15855260 Relationships: is a type of positive regulation of biosynthetic process [GO:0009891]; is a type of regulation of pyruvate decarboxylation to acetyl-CoA [GO:0010510]; is a type of positive regulation of amide metabolic process [GO:0034250]; is a type of positive regulation of phosphate metabolic process [GO:0045937]; is a type of positive regulation of small molecule metabolic process [GO:0062013]; positively regulates pyruvate decarboxylation to acetyl-CoA [GO:0006086] Definition: Any process that activates or increases the frequency, rate or extent of the chemical reactions and pathways resulting in the formation of acetyl-CoA from pyruvate. In most organisms, this pathway links glycolysis to the TCA cycle, by a series of three reactions carried out by a multisubunit complex called the 'pyruvate dehydrogenase complex', even though pyruvate dehydrogenase activity describes only one of those reactions.